{
  "gene": "UniProtKB:Q9H2L5",
  "gene_symbol": "RASSF4",
  "term_label": "Unknown molecular function",
  "gene_name": "Ras association domain-containing protein 4",
  "term_id": "UNKNOWN:0001"
}